fatty-acyl-CoA catabolic process [GO:0036115] (BP) Definition: The chemical reactions and pathways resulting in the breakdown of a fatty-acyl-CoA, any derivative of coenzyme A in which the sulfhydryl group is in thiolester linkage with a fatty-acyl group. Also known as: fatty-acyl-CoA breakdown, fatty-acyl-CoA catabolism, fatty-acyl-CoA degradation Relationships: is a type of fatty-acyl-CoA metabolic process [GO:0035337]; is_a sulfur compound catabolic process [GO:0044273]; is a type of purine-containing compound catabolic process [GO:0072523]; is a type of nucleoside phosphate catabolic process [GO:1901292]; is a type of fatty acid derivative catabolic process [GO:1901569] Subtypes: very long-chain fatty-acyl-CoA catabolic process [GO:0036113], medium-chain fatty-acyl-CoA catabolic process [GO:0036114], long-chain fatty-acyl-CoA catabolic process [GO:0036116], butyryl-CoA catabolic process [GO:0044580], 2-methylbutanoyl-CoA(4-) catabolic process [GO:1902190], GO:1902193, isovaleryl-CoA(4-) catabolic process [GO:1902196], GO:1902199, propionyl-CoA catabolic process [GO:1902859] References: PMID:10578051